{
  "term_label": "Unknown biological process",
  "term_id": "UNKNOWN:0002",
  "gene": "UniProtKB:Q8TAP9",
  "gene_symbol": "MPLKIP",
  "gene_name": "M-phase-specific PLK1-interacting protein"
}